{
  "gene_name": "PRKCA-binding protein",
  "term_label": "synaptic vesicle",
  "gene_symbol": "PICK1",
  "term_id": "GO:0008021",
  "gene": "UniProtKB:Q9NRD5"
}